serotonin transport [GO:0006837] (biological process) Relationships: is a type of GO:0015844; is a type of organic hydroxy compound transport [GO:0015850] Sources: GOC:ai Subtypes: GO:0001820, serotonin uptake [GO:0051610] Definition: The directed movement of serotonin into, out of or within a cell, or between cells, by means of some agent such as a transporter or pore. Serotonin (5-hydroxytryptamine) is a monoamine neurotransmitter occurring in the peripheral and central nervous systems.